{
  "gene_name": "Selenoprotein F",
  "term_id": "UNKNOWN:0002",
  "gene": "UniProtKB:O60613",
  "term_label": "Unknown biological process",
  "gene_symbol": "SELENOF"
}